{
  "gene_symbol": "SMIM32",
  "term_id": "UNKNOWN:0003",
  "gene_name": "Small integral membrane protein 32",
  "gene": "UniProtKB:A0A1B0GUA5",
  "term_label": "Unknown cellular component"
}